{
  "term_id": "GO:0001525",
  "term_label": "angiogenesis",
  "gene_name": "Angiomotin-like protein 2",
  "gene": "UniProtKB:Q9Y2J4",
  "gene_symbol": "AMOTL2"
}